{
  "gene": "UniProtKB:Q9UNT1",
  "gene_name": "Rab-like protein 2B",
  "term_label": "GTPase activity",
  "term_id": "GO:0003924",
  "gene_symbol": "RABL2B"
}